{
  "term_label": "Unknown biological process",
  "term_id": "UNKNOWN:0002",
  "gene": "UniProtKB:Q9NZR2",
  "gene_name": "Low-density lipoprotein receptor-related protein 1B",
  "gene_symbol": "LRP1B"
}